{
  "gene": "UniProtKB:Q8N6F7",
  "term_id": "GO:2000402",
  "gene_name": "Germinal center-associated signaling and motility protein",
  "gene_symbol": "GCSAM",
  "term_label": "negative regulation of lymphocyte migration"
}